{
  "term_label": "Unknown cellular component",
  "gene": "UniProtKB:Q6PCB5",
  "gene_name": "Lysine-specific demethylase RSBN1L",
  "term_id": "UNKNOWN:0003",
  "gene_symbol": "RSBN1L"
}